{
  "term_label": "guanyl-nucleotide exchange factor activity",
  "gene": "UniProtKB:P15498",
  "gene_symbol": "VAV1",
  "gene_name": "Proto-oncogene vav",
  "term_id": "GO:0005085"
}